{
  "gene_name": "Bromodomain and WD repeat-containing protein 1",
  "term_label": "regulation of cell shape",
  "term_id": "GO:0008360",
  "gene_symbol": "BRWD1",
  "gene": "UniProtKB:Q9NSI6"
}